{
  "term_id": "GO:0003823",
  "gene_name": "Immunoglobulin V-set domain-containing protein (Fragment)",
  "gene": "UniProtKB:A0A0J9YW62",
  "term_label": "antigen binding",
  "gene_symbol": "A0A0J9YW62"
}